{
  "term_label": "regulation of transcription by RNA polymerase II",
  "gene": "UniProtKB:P17947",
  "gene_symbol": "SPI1",
  "term_id": "GO:0006357",
  "gene_name": "Transcription factor PU.1"
}